cell adhesion mediator activity [GO:0098631] (molecular function) Relationships: is a type of cell adhesion molecule binding [GO:0050839]; is part of cell adhesion [GO:0007155] Definition: The binding by a cell-adhesion protein on a cell surface to an adhesion molecule on another cell surface or an external substrate, to mediate adhesion of the cell to the external substrate or to another cell. Also known as: cell adhesion molecule, protein binding involved in cell adhesion Subtypes: cell adhesion receptor activity [GO:0004895], laminin receptor activity [GO:0005055], cell-cell adhesion mediator activity [GO:0098632], cell-matrix adhesion mediator activity [GO:0098634] Sources: GOC:vw, Wikipedia:Cell_adhesion